{
  "gene": "UniProtKB:P11245",
  "gene_symbol": "NAT2",
  "term_id": "GO:0004060",
  "gene_name": "Arylamine N-acetyltransferase 2",
  "term_label": "arylamine N-acetyltransferase activity"
}